{
  "gene_name": "Granulocyte-macrophage colony-stimulating factor receptor subunit alpha",
  "term_label": "growth hormone receptor activity",
  "term_id": "GO:0004903",
  "gene_symbol": "CSF2RA",
  "gene": "UniProtKB:P15509"
}